clathrin vesicle coat [GO:0030125] (cellular component) Sources: GOC:mah Subtypes: GO:0030128, clathrin coat of synaptic vesicle [GO:0030129], GO:0030130 Definition: A clathrin coat found on a vesicle. Relationships: is a type of clathrin coat [GO:0030118]; is a type of vesicle coat [GO:0030120]; is part of clathrin-coated vesicle membrane [GO:0030665]